{
  "gene_name": "Macrophage-stimulating protein receptor",
  "gene": "UniProtKB:Q04912",
  "gene_symbol": "MST1R",
  "term_id": "GO:0016477",
  "term_label": "cell migration"
}